{
  "gene_name": "Ribonuclease P_MRP protein subunit POP5",
  "term_id": "GO:0000172",
  "gene": "UniProtKB:Q969H6",
  "term_label": "ribonuclease MRP complex",
  "gene_symbol": "POP5"
}